N-terminal protein acetyltransferase complex [GO:0031414] (cellular component) Also known as: NAT complex Relationships: is a type of protein acetyltransferase complex [GO:0031248]; is part of cytoplasm [GO:0005737] Definition: A complex that catalyzes the transfer of an acetyl group to the N-terminal residue of a protein acceptor molecule. Sources: GOC:mah Subtypes: NatA complex [GO:0031415], NatB complex [GO:0031416], NatC complex [GO:0031417]